{
  "gene_name": "Cytochrome P450 2E1",
  "gene": "UniProtKB:P05181",
  "term_label": "cytoplasm",
  "gene_symbol": "CYP2E1",
  "term_id": "GO:0005737"
}